{
  "term_id": "GO:0048812",
  "term_label": "neuron projection morphogenesis",
  "gene": "UniProtKB:P55160",
  "gene_symbol": "NCKAP1L",
  "gene_name": "Nck-associated protein 1-like"
}